RNA polymerase III general transcription initiation factor activity [GO:0000995] (molecular function) Relationships: is a type of GO:0140223; is part of transcription by RNA polymerase III [GO:0006383] Also known as: RNA polymerase III general initiation factor activity, RNA polymerase III transcription factor activity, sequence-specific DNA binding, core RNA polymerase III binding transcription factor activity, sequence-specific DNA binding RNA polymerase III transcription factor activity, transcription factor activity, core RNA polymerase III binding Definition: A general transcription initiation factor activity that contributes to transcription start site selection and transcription initiation of genes transcribed by RNA polymerase III. Factors required for RNA polymerase III transcription initiation include TFIIIA, TFIIIB and TFIIIC. RNA polymerase III transcribes genes encoding short RNAs, including tRNAs, 5S rRNA, U6 snRNA, the short ncRNA component of RNases P, the mitochondrial RNA processing (MRP) RNA, the signal recognition particle SRP RNA, and in higher eukaryotes a number of micro and other small RNAs, though there is some variability across species as to whether a given small noncoding RNA is transcribed by RNA polymerase II or RNA polymerase III. References: PMID:12381659, PMID:17977614, PMID:20413673, PMID:27068803 Sources: GOC:txnOH-2018, Wikipedia:RNA_polymerase_III